{
  "gene": "UniProtKB:P17028",
  "term_label": "regulation of transcription by RNA polymerase II",
  "gene_symbol": "ZNF24",
  "term_id": "GO:0006357",
  "gene_name": "Zinc finger protein 24"
}